short-chain 2-methyl fatty acyl-CoA dehydrogenase activity [GO:0003853] (molecular function) Also known as: 2-methyl branched chain acyl-CoA dehydrogenase activity, 2-methylacyl-CoA dehydrogenase activity, 2-methylbutanoyl-CoA dehydrogenase activity, 2-methylpropanoyl-CoA dehydrogenase activity, branched-chain acyl-CoA dehydrogenase activity, isobutyryl-CoA:FAD oxidoreductase activity, 2-methyl-branched-chain-enoyl-CoA reductase activity Definition: Catalysis of the reaction: Catalysis of the reaction: a short-chain 2-methyl fatty acyl-CoA + H+ + oxidized [electron-transfer flavoprotein] = a short-chain (2E)-2-methyl-2-enoyl-CoA + reduced [electron-transfer flavoprotein]. Relationships: is a type of GO:0016937 References: PMID:10989435, PMID:6401712